positive regulation of tongue muscle cell differentiation [GO:2001037] (biological process) Relationships: is a type of positive regulation of skeletal muscle fiber differentiation [GO:1902811]; is a type of regulation of tongue muscle cell differentiation [GO:2001035]; positively regulates tongue muscle cell differentiation [GO:0035981] Definition: Any process that activates or increases the frequency, rate or extent of tongue muscle cell differentiation. Sources: GOC:obol